taurine dioxygenase complex [GO:1990205] (cellular component) Definition: A protein complex capable of catalyzing the conversion of taurine and alpha-ketoglutarate to sulfite, aminoacetaldehyde and succinate under sulfur or cysteine starvation conditions. Its expression is repressed by the presence of sulfate or cysteine. In E. coli it is a homodimer or homotetramer of the protein TauD. References: PMID:12741810 Sources: GOC:bhm Also known as: 2-aminoethanesulfonate dioxygenase complex, alpha-ketoglutarate-dependent taurine dioxygenase complex, TauD complex Relationships: is a type of oxidoreductase complex [GO:1990204]; is part of GO:0005829